somatic diversification of FREP-based immune receptors [GO:0002567] (biological process) Relationships: is a type of GO:0002200 Note: Note that this type of immune receptor has been found in snails (Pulmonata, ncbi_axonomy_id:6519), but may also be seen in other species. References: PMID:16102575 Sources: GOC:add Definition: The process that results in the generation of sequence diversity of the FREP-based immune receptors of snails.